response to leukotriene B4 [GO:1905389] (biological process) Definition: Any process that results in a change in state or activity of a cell or an organism (in terms of movement, secretion, enzyme production, gene expression, etc.) as a result of a leukotriene B4 stimulus. Also known as: response to LTB4 Relationships: is a type of response to fatty acid [GO:0070542] Subtypes: GO:1905390 References: PMID:14656734 Sources: GOC:TermGenie, GO_REF:0000071